{
  "gene": "UniProtKB:Q96E14",
  "gene_symbol": "RMI2",
  "term_id": "GO:0043007",
  "term_label": "maintenance of rDNA",
  "gene_name": "RecQ-mediated genome instability protein 2"
}